enteric smooth muscle cell differentiation [GO:0035645] (biological process) Sources: CL:0002504, GOC:BHF Definition: The process in which a relatively unspecialized cell acquires specialized features of a smooth muscle cell of the intestine. Relationships: is a type of smooth muscle cell differentiation [GO:0051145]; is part of digestive tract development [GO:0048565] Also known as: intestinal smooth muscle cell differentiation